{
  "gene_name": "Serine_threonine-protein phosphatase 2A 65 kDa regulatory subunit A alpha isoform",
  "gene_symbol": "PPP2R1A",
  "term_id": "GO:0005829",
  "term_label": "cytosol",
  "gene": "UniProtKB:P30153"
}